phospholipid transport [GO:0015914] (biological process) Definition: The directed movement of phospholipids into, out of or within a cell, or between cells, by means of some agent such as a transporter or pore. Phospholipids are any lipids containing phosphoric acid as a mono- or diester. Regulation: regulated by regulation of phospholipid transport [GO:2001138]; negatively regulated by negative regulation of phospholipid transport [GO:2001139]; positively regulated by positive regulation of phospholipid transport [GO:2001140] Relationships: is a type of lipid transport [GO:0006869]; is a type of organophosphate ester transport [GO:0015748] Subtypes: phospholipid transfer to membrane [GO:0006649], aminophospholipid transport [GO:0015917], phospholipid efflux [GO:0033700], phospholipid translocation [GO:0045332], lysophospholipid transport [GO:0051977], intermembrane phospholipid transfer [GO:0120010], isopentenyl pyrophosphate import into mitochondrion [GO:0170046], ceramide 1-phosphate transport [GO:1902389] Sources: GOC:ai